{
  "term_id": "GO:0050911",
  "term_label": "detection of chemical stimulus involved in sensory perception of smell",
  "gene_name": "Olfactory receptor 10C1",
  "gene": "UniProtKB:Q96KK4",
  "gene_symbol": "OR10C1"
}